adhesion of symbiont to host cell surface via host glycoprotein [GO:0141025] (biological process) References: PMID:12010488, PMID:15487949, PMID:17630833, PMID:29184850 Relationships: is a type of adhesion of symbiont to host cell [GO:0044650] Definition: The attachment of a symbiont to its host by binding to a glycoprotein on the host cell surface. The host is defined as the larger of the organisms involved in a symbiotic interaction.